{
  "gene_name": "Transmembrane protein 132D",
  "term_label": "membrane",
  "gene_symbol": "TMEM132D",
  "term_id": "GO:0016020",
  "gene": "UniProtKB:Q14C87"
}